sequence-specific single stranded DNA binding [GO:0098847] (molecular function) Relationships: is a type of GO:0003697; is a type of sequence-specific DNA binding [GO:0043565] References: PMID:9531483 Definition: Binding to single-stranded DNA of a specific nucleotide composition. Subtypes: GO:0043047